{
  "term_id": "GO:0016485",
  "gene_symbol": "PSEN2",
  "gene_name": "Presenilin-2",
  "gene": "UniProtKB:P49810",
  "term_label": "protein processing"
}